{
  "gene_symbol": "EHD2",
  "gene_name": "EH domain-containing protein 2",
  "term_label": "protein localization to plasma membrane",
  "gene": "UniProtKB:Q9NZN4",
  "term_id": "GO:0072659"
}